{
  "gene_name": "Thrombomodulin",
  "term_id": "UNKNOWN:0001",
  "gene_symbol": "THBD",
  "gene": "UniProtKB:P07204",
  "term_label": "Unknown molecular function"
}